{
  "gene_name": "Ras-related protein Rab-6A",
  "gene": "UniProtKB:P20340",
  "gene_symbol": "RAB6A",
  "term_label": "protein localization to Golgi membrane",
  "term_id": "GO:1903292"
}